{
  "gene": "UniProtKB:P0DV77",
  "term_id": "GO:0006357",
  "term_label": "regulation of transcription by RNA polymerase II",
  "gene_symbol": "TPRX2",
  "gene_name": "Tetrapeptide repeat homeobox protein 2"
}